{
  "gene_symbol": "DPY19L1",
  "gene_name": "Probable C-mannosyltransferase DPY19L1",
  "term_id": "GO:0005789",
  "gene": "UniProtKB:Q2PZI1",
  "term_label": "endoplasmic reticulum membrane"
}